UDP catabolic process [GO:0006256] (biological process) Definition: The chemical reactions and pathways resulting in the breakdown of UDP, uridine (5'-)diphosphate. Sources: ISBN:0198506732 Also known as: UDP breakdown, UDP catabolism, UDP degradation Relationships: is a type of pyrimidine ribonucleoside diphosphate catabolic process [GO:0009195]; is a type of pyrimidine ribonucleotide catabolic process [GO:0009222]; is a type of UDP metabolic process [GO:0046048]